{
  "gene_symbol": "USP17L3",
  "gene_name": "Ubiquitin carboxyl-terminal hydrolase 17-like protein 3",
  "term_id": "GO:0031647",
  "term_label": "regulation of protein stability",
  "gene": "UniProtKB:A6NCW0"
}